exon-exon junction complex assembly [GO:1903040] (biological process) References: PMID:17606899 Sources: GOC:TermGenie, GOC:sart, GO_REF:0000079 Relationships: is a type of GO:0065003 Also known as: EJC assembly, EJC formation, exon-exon junction complex formation Definition: The aggregation, arrangement and bonding together of a set of components to form an exon-exon junction complex.